{
  "term_label": "stereocilia ankle link complex",
  "gene_name": "PDZ domain-containing protein 7",
  "term_id": "GO:0002142",
  "gene": "UniProtKB:Q9H5P4",
  "gene_symbol": "PDZD7"
}